{
  "term_label": "cytoplasm",
  "term_id": "GO:0005737",
  "gene_name": "Myosin-10",
  "gene_symbol": "MYH10",
  "gene": "UniProtKB:P35580"
}